anterograde synaptic vesicle transport [GO:0048490] (biological process) Relationships: is a type of anterograde axonal transport [GO:0008089]; is a type of synaptic vesicle transport along microtubule [GO:0099517] Definition: The directed movement of synaptic vesicle along axonal microtubules from the cell body to the presynapse. Also known as: anterograde axonal transport of synaptic vesicle Sources: GOC:jid, GOC:lmg Regulation: regulated by regulation of anterograde synaptic vesicle transport [GO:1903742]; negatively regulated by negative regulation of anterograde synaptic vesicle transport [GO:1903743]; positively regulated by positive regulation of anterograde synaptic vesicle transport [GO:1903744]